{
  "term_label": "DNA-binding transcription factor activity, RNA polymerase II-specific",
  "term_id": "GO:0000981",
  "gene": "UniProtKB:Q99853",
  "gene_symbol": "FOXB1",
  "gene_name": "Forkhead box protein B1"
}